{
  "gene_symbol": "GALR3",
  "gene": "UniProtKB:O60755",
  "term_id": "GO:0004966",
  "gene_name": "Galanin receptor type 3",
  "term_label": "galanin receptor activity"
}